{
  "term_id": "GO:0035082",
  "gene": "UniProtKB:Q4G0X9",
  "gene_name": "Coiled-coil domain-containing protein 40",
  "term_label": "axoneme assembly",
  "gene_symbol": "CCDC40"
}